5-formyltetrahydrofolate transmembrane transporter activity [GO:0015231] (molecular function) Definition: Enables the transfer of 5-formyltetrahydrofolate, the formylated derivative of tetrahydrofolate, from one side of a membrane to the other. Sources: GOC:ai Also known as: 5-formyltetrahydrofolate transporter activity Relationships: is a type of carboxylic acid transmembrane transporter activity [GO:0046943]; is a type of modified amino acid transmembrane transporter activity [GO:0072349]; is part of 5-formyltetrahydrofolate transport [GO:0015885]